antioxidant activity [GO:0016209] (molecular function) Subtypes: glutathione-disulfide reductase (NADPH) activity [GO:0004362], peroxidase activity [GO:0004601], superoxide dismutase activity [GO:0004784], thioredoxin-disulfide reductase (NADPH) activity [GO:0004791], sulfiredoxin activity [GO:0032542], glutathione dehydrogenase (ascorbate) activity [GO:0045174], superoxide reductase activity [GO:0050605] Sources: ISBN:0198506732 Definition: Inhibition of the reactions brought about by dioxygen (O2) or peroxides. Usually the antioxidant is effective because it can itself be more easily oxidized than the substance protected. The term is often applied to components that can trap free radicals, thereby breaking the chain reaction that normally leads to extensive biological damage. Relationships: is a type of molecular_function [GO:0003674]; is part of cellular oxidant detoxification [GO:0098869]